neurosecretory vesicle [GO:1990008] (cellular component) Definition: A large cytoplasmic membrane-bounded vesicle with an electron dense granular core, up to 150-200 nm in diameter, found in neurosecretory cells in the hypothalamus. Sources: ISBN:0195065719, NIF_Subcellular:sao2031592629 Relationships: is a type of granular vesicle [GO:1990005]